icosanoid metabolic process [GO:0006690] (biological process) Definition: The chemical reactions and pathways involving icosanoids, any of a group of C20 polyunsaturated fatty acids. Subtypes: leukotriene metabolic process [GO:0006691], prostanoid metabolic process [GO:0006692], arachidonate metabolic process [GO:0019369], GO:0019372, icosanoid biosynthetic process [GO:0046456] Sources: GOC:ma Also known as: eicosanoid metabolic process, eicosanoid metabolism, icosanoid metabolism Relationships: is a type of carboxylic acid metabolic process [GO:0019752]